{
  "term_label": "cytoplasm",
  "term_id": "GO:0005737",
  "gene_name": "Cystatin-11",
  "gene": "UniProtKB:Q9H112",
  "gene_symbol": "CST11"
}